response to Thyroid stimulating hormone [GO:1904400] (biological process) Definition: Any process that results in a change in state or activity of a cell or an organism (in terms of movement, secretion, enzyme production, gene expression, etc.) as a result of a Thyroid stimulating hormone stimulus. Relationships: is_a response to glycoprotein [GO:1904587] Subtypes: GO:1904401 References: PMID:11238928 Sources: GOC:TermGenie, GO_REF:0000071